{
  "gene_symbol": "DLK1",
  "gene": "UniProtKB:P80370",
  "term_label": "negative regulation of Notch signaling pathway",
  "term_id": "GO:0045746",
  "gene_name": "Protein delta homolog 1"
}